{
  "term_id": "GO:0016925",
  "gene": "UniProtKB:Q8NF64",
  "term_label": "protein sumoylation",
  "gene_symbol": "ZMIZ2",
  "gene_name": "Zinc finger MIZ domain-containing protein 2"
}